Noc1p-Noc2p complex [GO:0030690] (CC) Relationships: is a type of Noc complex [GO:0030689]; is part of GO:0030686; is part of preribosome, large subunit precursor [GO:0030687] References: PMID:12446671 Definition: A heterodimer associated with 90S and 66S preribosomes. Predominantly, but not exclusively, nucleolar; involved in ribosomal large subunit biogenesis. Note: Noc complexes exhibit a dynamic intranuclear location; consider also annotating to 'nucleolus ; GO:0005730' and/or 'nucleoplasm ; GO:0005654'. Note that the term name uses Saccharomyces gene product names because no other names have yet arisen for this complex; the term nevertheless can be used for analogous complexes in other eukaryotes, and the name can be changed if better wording is found.